{
  "term_id": "GO:0046512",
  "gene_name": "Sphingosine kinase 1",
  "term_label": "sphingosine biosynthetic process",
  "gene": "UniProtKB:Q9NYA1",
  "gene_symbol": "SPHK1"
}